{
  "gene": "UniProtKB:Q8WY36",
  "term_id": "GO:0006357",
  "term_label": "regulation of transcription by RNA polymerase II",
  "gene_symbol": "BBX",
  "gene_name": "HMG box transcription factor BBX"
}